regulation of cell proliferation involved in tissue homeostasis [GO:0060784] (biological process) Definition: Any process that modulates the frequency, rate or extent of cell proliferation resulting in the maintenance of a steady-state number of cells within a tissue. Sources: GOC:dph Relationships: is a type of regulation of cell population proliferation [GO:0042127]; is part of homeostasis of number of cells within a tissue [GO:0048873]